{
  "gene_name": "Centromere protein T",
  "term_id": "GO:0000278",
  "gene_symbol": "CENPT",
  "term_label": "mitotic cell cycle",
  "gene": "UniProtKB:Q96BT3"
}